{
  "term_id": "GO:0043484",
  "gene_symbol": "MBNL3",
  "gene_name": "Muscleblind-like protein 3",
  "term_label": "regulation of RNA splicing",
  "gene": "UniProtKB:Q9NUK0"
}